{
  "gene_name": "Zinc finger protein 514",
  "term_label": "regulation of transcription by RNA polymerase II",
  "gene": "UniProtKB:Q96K75",
  "term_id": "GO:0006357",
  "gene_symbol": "ZNF514"
}